{
  "term_id": "UNKNOWN:0003",
  "gene_symbol": "CCDC197",
  "gene_name": "Uncharacterized protein CCDC197",
  "gene": "UniProtKB:Q8NCU1",
  "term_label": "Unknown cellular component"
}